regulation of defense response to insect [GO:2000068] (biological process) Relationships: is a type of GO:0002831; is a type of regulation of defense response [GO:0031347]; is a type of regulation of response to external stimulus [GO:0032101]; RO_0002211 defense response to insect [GO:0002213] Also known as: regulation of physiological defense response to insect Definition: Any process that modulates the frequency, rate or extent of defense response to insect. Subtypes: GO:1900366, positive regulation of defense response to insect [GO:1900367] Sources: GOC:obol